{
  "gene": "UniProtKB:Q6P1M3",
  "gene_symbol": "LLGL2",
  "term_id": "GO:0008593",
  "term_label": "regulation of Notch signaling pathway",
  "gene_name": "LLGL scribble cell polarity complex component 2"
}